negative regulation of establishment or maintenance of neuroblast polarity [GO:2000248] (BP) Definition: Any process that stops, prevents, or reduces the frequency, rate or extent of establishment or maintenance of neuroblast polarity. Also known as: negative regulation of establishment and/or maintenance of neuroblast cell polarity Sources: GOC:obol Relationships: is_a negative regulation of cell fate commitment [GO:0010454]; is a type of regulation of establishment or maintenance of cell polarity [GO:0032878]; is a type of negative regulation of asymmetric cell division [GO:0045769]; negatively regulates GO:0045196